{
  "gene": "UniProtKB:P15692",
  "gene_name": "Vascular endothelial growth factor A, long form",
  "term_id": "GO:0060754",
  "term_label": "positive regulation of mast cell chemotaxis",
  "gene_symbol": "VEGFA"
}